{
  "term_id": "GO:0140445",
  "term_label": "chromosome, telomeric repeat region",
  "gene": "UniProtKB:Q5UIP0",
  "gene_name": "Telomere-associated protein RIF1",
  "gene_symbol": "RIF1"
}